{
  "gene_symbol": "KRT5",
  "term_label": "keratinization",
  "term_id": "GO:0031424",
  "gene_name": "Keratin, type II cytoskeletal 5",
  "gene": "UniProtKB:P13647"
}